{
  "term_id": "GO:0031251",
  "gene_symbol": "PAN3",
  "term_label": "PAN complex",
  "gene_name": "PAN2-PAN3 deadenylation complex subunit PAN3",
  "gene": "UniProtKB:Q58A45"
}